{
  "gene_name": "F-box and leucine-rich protein 22",
  "term_label": "Unknown biological process",
  "gene": "UniProtKB:Q6P050",
  "term_id": "UNKNOWN:0002",
  "gene_symbol": "FBXL22"
}